intramolecular oxidoreductase activity, interconverting aldoses and ketoses [GO:0016861] (molecular function) Definition: Catalysis of an oxidation-reduction (redox) reaction in which the hydrogen donor and acceptor, which is an aldose or a ketose, are the same molecule, and no oxidized product appears. Subtypes: (4S)-4-hydroxy-5-phosphonooxypentane-2,3-dione isomerase activity [GO:0002952], 1-(5-phosphoribosyl)-5-[(5-phosphoribosylamino)methylideneamino]imidazole-4-carboxamide isomerase activity [GO:0003949], GO:0004110, glucose-6-phosphate isomerase activity [GO:0004347], mannose-6-phosphate isomerase activity [GO:0004476], phosphoribosylanthranilate isomerase activity [GO:0004640], ribose-5-phosphate isomerase activity [GO:0004751], triose-phosphate isomerase activity [GO:0004807], 4-deoxy-L-threo-5-hexosulose-uronate ketol-isomerase activity [GO:0008697], GO:0008733, L-fucose isomerase activity [GO:0008736], L-rhamnose isomerase activity [GO:0008740], D-allose 6-phosphate isomerase activity [GO:0008786], arabinose isomerase activity [GO:0008790], glucuronate isomerase activity [GO:0008880], hydroxypyruvate isomerase activity [GO:0008903], GO:0009045, arabinose-5-phosphate isomerase activity [GO:0019146], 6-phospho-3-hexuloisomerase activity [GO:0043800], GO:0043877, GO:0043917, GO:0046523, D-lyxose ketol-isomerase activity [GO:0047828], galactose-6-phosphate isomerase activity [GO:0050044], GO:0050089, ribose isomerase activity [GO:0050261], sulfoquinovose isomerase activity [GO:0061593], GO:0102482 Sources: EC:5.3.1.-, GOC:jl Also known as: intramolecular isomerase activity, interconverting aldoses and ketoses Relationships: is a type of intramolecular oxidoreductase activity [GO:0016860]